{
  "gene_symbol": "GRK6",
  "gene_name": "G protein-coupled receptor kinase 6",
  "gene": "UniProtKB:P43250",
  "term_id": "GO:0009966",
  "term_label": "regulation of signal transduction"
}